{
  "gene": "UniProtKB:Q8N8A8",
  "gene_name": "Protein FAM169BP",
  "gene_symbol": "FAM169BP",
  "term_id": "UNKNOWN:0001",
  "term_label": "Unknown molecular function"
}